{
  "gene_symbol": "PDXDC2P",
  "term_label": "Unknown biological process",
  "term_id": "UNKNOWN:0002",
  "gene_name": "Putative pyridoxal-dependent decarboxylase domain-containing protein 2",
  "gene": "UniProtKB:Q6P474"
}